{
  "term_label": "actin filament organization",
  "gene_symbol": "RHOF",
  "gene": "UniProtKB:Q9HBH0",
  "term_id": "GO:0007015",
  "gene_name": "Rho-related GTP-binding protein RhoF"
}